menstruation [GO:0042703] (biological process) Note: Note that this term should not be used for direct annotation. If you are trying to make an annotation to x phase, it is likely that the correct annotation is 'regulation of x/y phase transition' or to a process which occurs during the reported phase. To capture the phase when a specific location or process is observed, the phase term can be used in an annotation extension (PMID:24885854) applied to a cellular component term (with the relation exists_during) or a biological process term (with the relation happens_during). Relationships: is a type of GO:0022601 Definition: The cyclic, physiologic discharge through the vagina of blood and endometrial tissues from the nonpregnant uterus. References: PMID:8693059 Sources: GOC:curators